{
  "gene": "UniProtKB:Q6UXB2",
  "gene_symbol": "CXCL17",
  "term_label": "extracellular space",
  "term_id": "GO:0005615",
  "gene_name": "C-X-C motif chemokine 17"
}